glycine:2-oxoglutarate aminotransferase activity [GO:0047958] (molecular function) Definition: Catalysis of the reaction: glycine + 2-oxoglutarate = glyoxylate + L-glutamate. Also known as: glycine aminotransferase activity, glycine transaminase activity, L-glutamate:glyoxylate aminotransferase activity, glutamate-glyoxylate transaminase activity, glutamic-glyoxylic transaminase activity, glyoxylate-glutamate aminotransferase activity, glyoxylate-glutamic transaminase activity Relationships: is a type of transaminase activity [GO:0008483] Sources: EC:2.6.1.4, MetaCyc:GLYCINE-AMINOTRANSFERASE-RXN